{
  "gene_name": "Cdc42 effector protein 5",
  "gene": "UniProtKB:Q6NZY7",
  "gene_symbol": "CDC42EP5",
  "term_id": "GO:0007266",
  "term_label": "Rho protein signal transduction"
}